{
  "gene": "UniProtKB:A0A1W2PR64",
  "gene_symbol": "TAF11L9",
  "gene_name": "TATA-box-binding protein-associated factor 11-like protein 9",
  "term_label": "transcription factor TFIID complex",
  "term_id": "GO:0005669"
}